actin filament binding [GO:0051015] (molecular function) Subtypes: actin lateral binding [GO:0003786] Regulation: negatively regulated by negative regulation of actin filament binding [GO:1904530]; positively regulated by positive regulation of actin filament binding [GO:1904531] Sources: ISBN:0198506732 Relationships: is a type of actin binding [GO:0003779]; is a type of protein-containing complex binding [GO:0044877] Also known as: F-actin binding, actin cross-linking activity Definition: Binding to an actin filament, also known as F-actin, a helical filamentous polymer of globular G-actin subunits.